immunoglobulin-mediated neutralization [GO:0097282] (biological process) Sources: GOC:add, GOC:rv Relationships: is a type of immunoglobulin mediated immune response [GO:0016064]; has part GO:0003823 Definition: The inhibition of an antigen's biological effects by antibody binding to it. An example is neutralization of diphtheria toxin by preventing its entry into human cells via the binding of antibody specific for diphtheria toxin. Also known as: antibody-mediated neutralization